{
  "gene_symbol": "HOXD10",
  "gene": "UniProtKB:P28358",
  "term_id": "GO:0005634",
  "gene_name": "Homeobox protein Hox-D10",
  "term_label": "nucleus"
}